{
  "term_id": "GO:0008270",
  "gene_name": "Transmembrane protein 163",
  "gene": "UniProtKB:Q8TC26",
  "term_label": "zinc ion binding",
  "gene_symbol": "TMEM163"
}